{
  "gene_symbol": "ZNF682",
  "gene": "UniProtKB:O95780",
  "term_label": "Unknown cellular component",
  "gene_name": "Zinc finger protein 682",
  "term_id": "UNKNOWN:0003"
}